dimethylglycine oxidase activity [GO:0047866] (molecular function) Also known as: N,N-dimethylglycine:oxygen oxidoreductase (demethylating) Sources: EC:1.5.3.10, RHEA:17077 Definition: Catalysis of the reaction: N,N-dimethylglycine + H2O + O2 = formaldehyde + H2O2 + sarcosine. Relationships: is a type of oxidoreductase activity, acting on the CH-NH group of donors, oxygen as acceptor [GO:0016647]